{
  "gene_name": "BRD4-interacting chromatin-remodeling complex-associated protein-like",
  "gene_symbol": "BICRAL",
  "gene": "UniProtKB:Q6AI39",
  "term_label": "SWI/SNF complex",
  "term_id": "GO:0016514"
}